{
  "gene": "UniProtKB:Q9BZ95",
  "gene_symbol": "NSD3",
  "term_label": "regulation of DNA-templated transcription",
  "term_id": "GO:0006355",
  "gene_name": "Histone-lysine N-methyltransferase NSD3"
}